{
  "gene_symbol": "TBX5",
  "gene_name": "T-box transcription factor TBX5",
  "term_label": "chromatin",
  "term_id": "GO:0000785",
  "gene": "UniProtKB:Q99593"
}